{
  "term_label": "Unknown biological process",
  "gene_name": "Protein-lysine N-methyltransferase EEF2KMT",
  "term_id": "UNKNOWN:0002",
  "gene": "UniProtKB:Q96G04",
  "gene_symbol": "EEF2KMT"
}